{
  "gene_name": "Non-receptor tyrosine-protein kinase TYK2",
  "gene_symbol": "TYK2",
  "term_label": "cytosol",
  "term_id": "GO:0005829",
  "gene": "UniProtKB:P29597"
}